{
  "gene_symbol": "SMDT1",
  "gene_name": "Essential MCU regulator, mitochondrial",
  "gene": "UniProtKB:Q9H4I9",
  "term_label": "Unknown molecular function",
  "term_id": "UNKNOWN:0001"
}